{
  "gene_name": "Adhesion G-protein coupled receptor G5",
  "gene": "UniProtKB:Q8IZF4",
  "term_label": "plasma membrane",
  "gene_symbol": "ADGRG5",
  "term_id": "GO:0005886"
}